{
  "term_label": "mitochondrion",
  "term_id": "GO:0005739",
  "gene": "UniProtKB:P13196",
  "gene_name": "5-aminolevulinate synthase, non-specific, mitochondrial",
  "gene_symbol": "ALAS1"
}